regulation of apoptotic process involved in morphogenesis [GO:1902337] (biological process) Relationships: is a type of regulation of apoptotic process involved in development [GO:1904748]; regulates GO:0060561 References: PMID:12202035 Sources: GOC:TermGenie, GOC:sart Definition: Any process that modulates the frequency, rate or extent of apoptotic process involved in morphogenesis. Also known as: regulation of apoptosis involved in morphogenesis, regulation of apoptosis involved in development, regulation of morphogenetic apoptosis Subtypes: GO:0072039, GO:1902256, GO:1902338, positive regulation of apoptotic process involved in morphogenesis [GO:1902339]